{
  "gene_name": "Tektin-3",
  "gene": "UniProtKB:Q9BXF9",
  "term_id": "GO:0015630",
  "gene_symbol": "TEKT3",
  "term_label": "microtubule cytoskeleton"
}